{
  "term_label": "Unknown molecular function",
  "term_id": "UNKNOWN:0001",
  "gene_name": "Putative protein BCE-1",
  "gene_symbol": "BCE1",
  "gene": "UniProtKB:O60756"
}